ornithine-acyl [acyl carrier protein] N-acyltransferase activity [GO:0043810] (molecular function) Definition: Catalysis of the reaction: (3R)-3-hydroxyacyl-[acyl-carrier protein] + L-ornithine = lyso-ornithine lipid + [acyl-carrier protein]. The enzyme, found in bacteria, catalyzes the first step in the biosynthesis of ornithine lipids. Also known as: L-ornithine N(alpha)-acyltransferase, ornithine-acyl[acyl carrier protein] N-acyltransferase activity Relationships: is a type of N-acyltransferase activity [GO:0016410] References: PMID:15341653 Sources: RHEA:20633